{
  "gene_symbol": "NAGS",
  "gene": "UniProtKB:Q8N159",
  "term_label": "mitochondrial matrix",
  "gene_name": "N-acetylglutamate synthase, mitochondrial",
  "term_id": "GO:0005759"
}